regulation of radial pattern formation [GO:0090213] (biological process) Also known as: regulation of radial pattern specification Definition: Any process that modulates the rate, frequency or extent of radial pattern formation, the regionalization process that results in defined areas around a point in which specific types of cell differentiation will occur. Relationships: is a type of regulation of multicellular organismal process [GO:0051239]; regulates radial pattern formation [GO:0009956] Sources: GOC:tb